{
  "gene": "UniProtKB:Q8TE67",
  "gene_name": "Epidermal growth factor receptor kinase substrate 8-like protein 3",
  "term_label": "plasma membrane",
  "term_id": "GO:0005886",
  "gene_symbol": "EPS8L3"
}